{
  "gene": "UniProtKB:Q12849",
  "term_label": "regulation of RNA splicing",
  "gene_symbol": "GRSF1",
  "gene_name": "G-rich sequence factor 1",
  "term_id": "GO:0043484"
}